{
  "term_id": "GO:0099550",
  "gene_name": "Complement C1q-like protein 3",
  "term_label": "trans-synaptic signaling, modulating synaptic transmission",
  "gene": "UniProtKB:Q5VWW1",
  "gene_symbol": "C1QL3"
}